{
  "term_label": "Unknown molecular function",
  "gene_symbol": "PDGFRL",
  "gene_name": "Platelet-derived growth factor receptor-like protein",
  "gene": "UniProtKB:Q15198",
  "term_id": "UNKNOWN:0001"
}